{
  "gene_name": "OCIA domain-containing protein 1",
  "gene_symbol": "OCIAD1",
  "term_label": "Unknown biological process",
  "term_id": "UNKNOWN:0002",
  "gene": "UniProtKB:Q9NX40"
}